{
  "term_id": "GO:0000978",
  "gene": "UniProtKB:Q8N587",
  "gene_name": "Zinc finger protein 561",
  "term_label": "RNA polymerase II cis-regulatory region sequence-specific DNA binding",
  "gene_symbol": "ZNF561"
}